{
  "term_label": "endoplasmic reticulum membrane",
  "term_id": "GO:0005789",
  "gene_name": "GPI mannosyltransferase 4",
  "gene": "UniProtKB:Q86VD9",
  "gene_symbol": "PIGZ"
}